{
  "gene_name": "Biorientation of chromosomes in cell division protein 1",
  "term_label": "Unknown cellular component",
  "gene_symbol": "BOD1",
  "gene": "UniProtKB:Q96IK1",
  "term_id": "UNKNOWN:0003"
}